{
  "term_id": "GO:0007188",
  "gene": "UniProtKB:P41587",
  "gene_name": "Vasoactive intestinal polypeptide receptor 2",
  "term_label": "adenylate cyclase-modulating G protein-coupled receptor signaling pathway",
  "gene_symbol": "VIPR2"
}